{
  "term_label": "protein O-linked glycosylation",
  "gene": "UniProtKB:Q6IS24",
  "gene_symbol": "GALNT17",
  "gene_name": "Polypeptide N-acetylgalactosaminyltransferase 17",
  "term_id": "GO:0006493"
}